{
  "gene_name": "UL16-binding protein 2",
  "term_id": "GO:0042267",
  "gene": "UniProtKB:Q9BZM5",
  "term_label": "natural killer cell mediated cytotoxicity",
  "gene_symbol": "ULBP2"
}